DNA-templated transcription [GO:0006351] (biological process) Relationships: is a type of GO:0032774; is part of gene expression [GO:0010467] Sources: GOC:jl, GOC:txnOH Subtypes: transcription by RNA polymerase IV [GO:0001059], transcription by RNA polymerase V [GO:0001060], transcription by RNA polymerase I [GO:0006360], GO:0006366, GO:0006383, mitochondrial transcription [GO:0006390], mRNA transcription [GO:0009299], GO:0009300, snRNA transcription [GO:0009301], sno(s)RNA transcription [GO:0009302], rRNA transcription [GO:0009303], GO:0009304, plastid transcription [GO:0042793], miRNA transcription [GO:0061614], telomeric repeat-containing RNA transcription [GO:0097393], GO:0140541, lncRNA transcription [GO:0140742] Also known as: cellular transcription, transcription, DNA-dependent transcription, transcription, DNA-dependent, transcription, DNA-templated, bacterial transcription, transcription from bacterial-type RNA polymerase promoter Regulation: regulated by regulation of DNA-templated transcription [GO:0006355]; negatively regulated by negative regulation of DNA-templated transcription [GO:0045892]; positively regulated by positive regulation of DNA-templated transcription [GO:0045893] Definition: The synthesis of an RNA transcript from a DNA template.